{
  "term_id": "GO:0005686",
  "gene_name": "Putative small nuclear ribonucleoprotein G-like protein 15",
  "gene_symbol": "SNRPGP15",
  "term_label": "U2 snRNP",
  "gene": "UniProtKB:A8MWD9"
}